{
  "gene_symbol": "VPS37B",
  "gene": "UniProtKB:Q9H9H4",
  "term_id": "GO:0000813",
  "term_label": "ESCRT I complex",
  "gene_name": "Vacuolar protein sorting-associated protein 37B"
}